{
  "gene_symbol": "CSNK2A1",
  "gene_name": "Casein kinase II subunit alpha",
  "term_id": "GO:0051726",
  "gene": "UniProtKB:P68400",
  "term_label": "regulation of cell cycle"
}